{
  "term_id": "GO:0000785",
  "term_label": "chromatin",
  "gene_symbol": "KDM3A",
  "gene": "UniProtKB:Q9Y4C1",
  "gene_name": "Lysine-specific demethylase 3A"
}